{
  "gene": "UniProtKB:Q7L266",
  "gene_name": "Isoaspartyl peptidase_L-asparaginase",
  "gene_symbol": "ASRGL1",
  "term_id": "GO:0008798",
  "term_label": "beta-aspartyl-peptidase activity"
}